{
  "gene_symbol": "PLK1",
  "term_label": "kinetochore",
  "gene_name": "Serine_threonine-protein kinase PLK1",
  "term_id": "GO:0000776",
  "gene": "UniProtKB:P53350"
}